{
  "term_id": "GO:0008260",
  "gene_name": "Succinyl-CoA:3-ketoacid coenzyme A transferase 1, mitochondrial",
  "gene_symbol": "OXCT1",
  "term_label": "succinyl-CoA:3-oxo-acid CoA-transferase activity",
  "gene": "UniProtKB:P55809"
}